{
  "gene_name": "Protocadherin alpha-3",
  "gene": "UniProtKB:Q9Y5H8",
  "term_label": "cell adhesion",
  "term_id": "GO:0007155",
  "gene_symbol": "PCDHA3"
}